{
  "gene": "UniProtKB:Q9Y3B4",
  "term_id": "UNKNOWN:0001",
  "term_label": "Unknown molecular function",
  "gene_symbol": "SF3B6",
  "gene_name": "Splicing factor 3B subunit 6"
}